{
  "gene_symbol": "HIPK1",
  "term_id": "GO:0005737",
  "gene": "UniProtKB:Q86Z02",
  "gene_name": "Homeodomain-interacting protein kinase 1",
  "term_label": "cytoplasm"
}